{
  "gene_name": "Fanconi anemia group G protein",
  "gene": "UniProtKB:O15287",
  "gene_symbol": "FANCG",
  "term_label": "Unknown molecular function",
  "term_id": "UNKNOWN:0001"
}